{
  "term_id": "UNKNOWN:0003",
  "gene_name": "Putative uncharacterized protein encoded by LINC00310",
  "gene_symbol": "LINC00310",
  "term_label": "Unknown cellular component",
  "gene": "UniProtKB:P59036"
}